myoblast fate specification [GO:0048626] (biological process) Relationships: is a type of cell fate specification [GO:0001708]; is part of myoblast fate commitment [GO:0048625] Subtypes: myoblast fate specification involved in skeletal muscle regeneration [GO:0014838] Definition: The process in which a cell becomes capable of differentiating autonomously into a myoblast in an environment that is neutral with respect to the developmental pathway. Upon specification, the cell fate can be reversed. A myoblast is a mononucleate cell type that, by fusion with other myoblasts, gives rise to the myotubes that eventually develop into skeletal muscle fibers. Sources: CL:0000056, GOC:dph, GOC:mtg_muscle